negative regulation of corticotropin secretion [GO:0051460] (biological process) Sources: GOC:ai Definition: Any process that stops, prevents, or reduces the frequency, rate or extent of the regulated release of corticotropic hormone from a cell. Also known as: down regulation of adrenocorticotropin secretion, down-regulation of adrenocorticotropin secretion, downregulation of adrenocorticotropin secretion, negative regulation of ACTH secretion, negative regulation of adrenocorticotropic hormone secretion, negative regulation of adrenocorticotropin secretion, negative regulation of adrenotropic hormone secretion, negative regulation of adrenotropin secretion, negative regulation of corticotropic hormone secretion, inhibition of adrenocorticotropin secretion Relationships: is a type of negative regulation of multicellular organismal process [GO:0051241]; is_a regulation of corticotropin secretion [GO:0051459]; is a type of negative regulation of peptide hormone secretion [GO:0090278]; negatively regulates corticotropin secretion [GO:0051458]